negative regulation of adult chitin-containing cuticle pigmentation [GO:0048083] (biological process) Sources: GOC:jid, GOC:mtg_sensu Definition: Any process that stops, prevents, or reduces the frequency, rate or extent of establishment of the adult pattern of pigmentation in the cuticle of an organism. Also known as: down regulation of adult chitin-containing cuticle pigmentation, down-regulation of adult chitin-containing cuticle pigmentation, downregulation of adult chitin-containing cuticle pigmentation, inhibition of adult chitin-containing cuticle pigmentation Relationships: is a type of GO:0045800; is a type of negative regulation of cuticle pigmentation [GO:0048080]; is a type of regulation of adult chitin-containing cuticle pigmentation [GO:0048082]; negatively regulates GO:0048085